O-linoleoyltransferase activity [GO:0032576] (molecular function) Definition: Catalysis of the transfer of a linoleoyl ((9Z,12Z)-octadeca-9,12-dienoyl) group to an oxygen atom on the acceptor molecule. Relationships: is a type of O-acyltransferase activity [GO:0008374] Subtypes: phosphatidylcholine:cardiolipin O-linoleoyltransferase activity [GO:0032577] Sources: GOC:cb